polyterpenoid biosynthetic process [GO:0016112] (biological process) Also known as: polyterpenoid anabolism, polyterpenoid biosynthesis, polyterpenoid formation, polyterpenoid synthesis, polyterpene biosynthesis, polyterpene biosynthetic process Sources: GOC:go_curators Relationships: is a type of GO:0016114 Definition: The chemical reactions and pathways resulting in the formation of polyterpenoid compounds, terpenoids with more than eight isoprene units.